{
  "term_id": "GO:0004869",
  "term_label": "cysteine-type endopeptidase inhibitor activity",
  "gene_symbol": "KNG1",
  "gene": "UniProtKB:P01042",
  "gene_name": "Kininogen-1"
}